{
  "gene": "UniProtKB:Q96GA7",
  "term_id": "GO:0006565",
  "gene_symbol": "SDSL",
  "gene_name": "Serine dehydratase-like",
  "term_label": "L-serine catabolic process"
}